{
  "term_label": "plasma membrane",
  "gene": "UniProtKB:Q96QS1",
  "gene_name": "Tetraspanin-32",
  "gene_symbol": "TSPAN32",
  "term_id": "GO:0005886"
}